{
  "term_label": "tricellular tight junction",
  "term_id": "GO:0061689",
  "gene": "UniProtKB:Q86X29",
  "gene_name": "Lipolysis-stimulated lipoprotein receptor",
  "gene_symbol": "LSR"
}